{
  "gene_name": "Translocator protein 2",
  "gene_symbol": "TSPO2",
  "term_label": "Unknown biological process",
  "term_id": "UNKNOWN:0002",
  "gene": "UniProtKB:Q5TGU0"
}